{
  "gene_name": "Glutamate dehydrogenase 1, mitochondrial",
  "gene": "UniProtKB:P00367",
  "term_id": "GO:0006538",
  "gene_symbol": "GLUD1",
  "term_label": "L-glutamate catabolic process"
}